{
  "term_label": "regulation of transcription by RNA polymerase II",
  "gene": "UniProtKB:Q92570",
  "term_id": "GO:0006357",
  "gene_name": "Nuclear receptor subfamily 4 group A member 3",
  "gene_symbol": "NR4A3"
}